{
  "gene_symbol": "CCNE1",
  "gene": "UniProtKB:P24864",
  "term_id": "GO:0000082",
  "gene_name": "G1_S-specific cyclin-E1",
  "term_label": "G1/S transition of mitotic cell cycle"
}